positive regulation of protein kinase C activity [GO:1900020] (biological process) Sources: GOC:TermGenie, GOC:signaling Relationships: is a type of GO:0071902; is a type of regulation of protein kinase C activity [GO:1900019]; positively regulates GO:0004697 Also known as: positive regulation of PKC activity, up regulation of PKC activity, positive regulation of PKC, up regulation of PKC Definition: Any process that activates or increases the frequency, rate or extent of protein kinase C activity.